smooth muscle adaptation [GO:0014805] (BP) Relationships: is a type of muscle adaptation [GO:0043500] Definition: Any process in which smooth muscle adapts, with consequent modifications to structural and/or functional phenotypes, in response to a stimulus. Stimuli include contractile activity, loading conditions, substrate supply, and environmental factors. These adaptive events occur in both muscle fibers and associated structures (motoneurons and capillaries), and they involve alterations in regulatory mechanisms, contractile properties and metabolic capacities. Subtypes: GO:0014806, smooth muscle atrophy [GO:0014890], GO:0014895 Also known as: smooth muscle plasticity Sources: GOC:mtg_muscle